homodimeric serine palmitoyltransferase complex [GO:0002179] (cellular component) Relationships: is a type of palmitoyltransferase complex [GO:0002178] Note: This complex occurs primarily in bacteria. Sources: GOC:hjd Definition: A homodimeric complex which transfers a palmitoyl group onto serine, forming 3-dehydro-D-sphinganine.